{
  "gene": "UniProtKB:P01730",
  "gene_name": "T-cell surface glycoprotein CD4",
  "gene_symbol": "CD4",
  "term_id": "GO:0001618",
  "term_label": "virus receptor activity"
}